{
  "gene_name": "DNA-directed RNA polymerase II subunit RPB2",
  "term_label": "Unknown molecular function",
  "gene": "UniProtKB:P30876",
  "term_id": "UNKNOWN:0001",
  "gene_symbol": "POLR2B"
}